{
  "term_label": "box C/D methylation guide snoRNP complex binding",
  "term_id": "GO:0062064",
  "gene": "UniProtKB:Q8N5I9",
  "gene_name": "NOP protein chaperone 1",
  "gene_symbol": "NOPCHAP1"
}